{
  "gene": "UniProtKB:P35226",
  "gene_name": "Polycomb complex protein BMI-1",
  "gene_symbol": "BMI1",
  "term_label": "PRC1 complex",
  "term_id": "GO:0035102"
}